TAF4B-containing transcription factor TFIID complex [GO:0070556] (CC) Also known as: TFIID complex, B-cell specific Relationships: is a type of transcription factor TFIID complex [GO:0005669] References: PMID:8858156 Sources: GOC:mah Definition: A transcription factor TFIID complex that contains the TBP-associated factor TAF4B (also known as TAFII105 in human), a cell-type-specific variant of TAF4.